{
  "gene": "UniProtKB:Q9BZQ8",
  "gene_symbol": "NIBAN1",
  "term_label": "Unknown biological process",
  "term_id": "UNKNOWN:0002",
  "gene_name": "Protein Niban 1"
}